{
  "gene_name": "GA-binding protein alpha chain",
  "term_label": "nucleus",
  "term_id": "GO:0005634",
  "gene_symbol": "GABPA",
  "gene": "UniProtKB:Q06546"
}